{
  "gene_symbol": "RAC3",
  "term_id": "GO:0016601",
  "gene_name": "Ras-related C3 botulinum toxin substrate 3",
  "gene": "UniProtKB:P60763",
  "term_label": "Rac protein signal transduction"
}